{
  "gene": "UniProtKB:P41226",
  "gene_symbol": "UBA7",
  "term_label": "cytoplasm",
  "gene_name": "Ubiquitin-like modifier-activating enzyme 7",
  "term_id": "GO:0005737"
}